{
  "gene_symbol": "IRAG1",
  "term_id": "UNKNOWN:0003",
  "term_label": "Unknown cellular component",
  "gene_name": "Inositol 1,4,5-triphosphate receptor associated 1",
  "gene": "UniProtKB:Q9Y6F6"
}